{
  "gene_name": "Dicarboxylate carrier SLC25A8",
  "gene_symbol": "UCP2",
  "term_id": "GO:0015078",
  "term_label": "proton transmembrane transporter activity",
  "gene": "UniProtKB:P55851"
}